protein nitrosylation [GO:0017014] (BP) Also known as: protein amino acid nitrosylation Definition: The covalent addition of a nitric oxide group to an amino acid within a protein. References: PMID:20972426 Sources: GOC:ai Subtypes: peptidyl-cysteine S-nitrosylation [GO:0018119] Relationships: is a type of protein modification process [GO:0036211]